pelvic fin morphogenesis [GO:0035139] (biological process) Sources: GOC:dgh Relationships: is a type of fin morphogenesis [GO:0033334]; is part of GO:0033340 Subtypes: embryonic pelvic fin morphogenesis [GO:0035119], post-embryonic pelvic fin morphogenesis [GO:0035131] Definition: The process in which the anatomical structures of the pelvic fin are generated and organized. Pelvic fins are bilaterally paired fins mounted in a ventral-lateral position on most fish. These fins are used primarily for lateral mobility and propulsion.